{
  "term_label": "cleavage furrow",
  "term_id": "GO:0032154",
  "gene_name": "Abscission_NoCut checkpoint regulator",
  "gene_symbol": "ZFYVE19",
  "gene": "UniProtKB:Q96K21"
}